metanephric glomerular basement membrane development [GO:0072274] (biological process) Sources: GOC:mtg_kidney_jan10 Definition: The process whose specific outcome is the progression of the metanephric glomerular basement membrane over time, from its formation to the mature structure. The metanephric glomerular basement membrane is the basal laminal portion of the metanephric glomerulus which performs the actual filtration. Relationships: is a type of glomerular basement membrane development [GO:0032836]; is part of metanephric glomerulus development [GO:0072224]